syncytiotrophoblast cell differentiation involved in labyrinthine layer development [GO:0060715] (biological process) Sources: GOC:dph Relationships: is a type of cell differentiation involved in embryonic placenta development [GO:0060706]; is part of labyrinthine layer development [GO:0060711] Definition: The process in which a chorionic trophoblast cell acquires specialized features of a syncytiotrophoblast of the labyrinthine layer of the placenta.